{
  "term_id": "GO:0038092",
  "term_label": "nodal signaling pathway",
  "gene_name": "Teratocarcinoma-derived growth factor 1",
  "gene": "UniProtKB:P13385",
  "gene_symbol": "TDGF1"
}